{
  "gene": "UniProtKB:Q8NGY5",
  "gene_name": "Olfactory receptor 6N1",
  "term_label": "detection of chemical stimulus involved in sensory perception of smell",
  "term_id": "GO:0050911",
  "gene_symbol": "OR6N1"
}